insulin-like growth factor receptor binding [GO:0005159] (molecular function) Sources: GOC:jl Relationships: is a type of signaling receptor binding [GO:0005102] Definition: Binding to an insulin-like growth factor receptor. Also known as: IGF receptor binding, insulin-like growth factor, insulin-like growth factor receptor ligand